{
  "gene": "UniProtKB:Q9BSU1",
  "term_label": "dendrite",
  "gene_symbol": "PHAF1",
  "gene_name": "Phagosome assembly factor 1",
  "term_id": "GO:0030425"
}